{
  "term_label": "Unknown cellular component",
  "gene_name": "Calcium-binding protein 39",
  "term_id": "UNKNOWN:0003",
  "gene_symbol": "CAB39",
  "gene": "UniProtKB:Q9Y376"
}